{
  "term_id": "UNKNOWN:0003",
  "term_label": "Unknown cellular component",
  "gene_name": "Coiled-coil domain-containing protein 179",
  "gene": "UniProtKB:H3BU77",
  "gene_symbol": "CCDC179"
}